{
  "term_label": "Unknown biological process",
  "gene_name": "CHD9 neighbor protein",
  "gene": "UniProtKB:A0A1B0GV96",
  "term_id": "UNKNOWN:0002",
  "gene_symbol": "CHD9NB"
}